poly(A)-specific ribonuclease activity [GO:0004535] (molecular function) Sources: EC:3.1.13.4, ISBN:0198547684 Relationships: is a type of 3'-5'-RNA exonuclease activity [GO:0000175] Definition: Catalysis of the exonucleolytic cleavage of poly(A) to 5'-AMP. Also known as: poly(A)-specific RNase activity, 2',3'-exoribonuclease activity, 3'-exoribonuclease activity